{
  "term_id": "UNKNOWN:0002",
  "gene_name": "E3 ubiquitin-protein ligase RNF187",
  "gene": "UniProtKB:Q5TA31",
  "term_label": "Unknown biological process",
  "gene_symbol": "RNF187"
}